{
  "term_id": "GO:0031663",
  "term_label": "lipopolysaccharide-mediated signaling pathway",
  "gene_name": "Interleukin-1 receptor-associated kinase 4",
  "gene": "UniProtKB:Q9NWZ3",
  "gene_symbol": "IRAK4"
}